{
  "gene": "UniProtKB:Q9UHA2",
  "gene_symbol": "SS18L2",
  "term_label": "Unknown biological process",
  "term_id": "UNKNOWN:0002",
  "gene_name": "SS18-like protein 2"
}